{
  "gene": "UniProtKB:Q15561",
  "term_label": "embryonic organ development",
  "gene_symbol": "TEAD4",
  "term_id": "GO:0048568",
  "gene_name": "Transcriptional enhancer factor TEF-3"
}